{
  "gene_name": "A-kinase anchor protein 5",
  "term_id": "GO:0034237",
  "term_label": "protein kinase A regulatory subunit binding",
  "gene": "UniProtKB:P24588",
  "gene_symbol": "AKAP5"
}